synapse maturation [GO:0060074] (biological process) Regulation: regulated by regulation of synapse maturation [GO:0090128]; positively regulated by positive regulation of synapse maturation [GO:0090129]; negatively regulated by GO:2000297 Also known as: synaptic maturation Sources: GOC:dph, GOC:ef Definition: The process that organizes a synapse so that it attains its fully functional state. Synaptic maturation plays a critical role in the establishment of effective synaptic connections in early development. Relationships: is a type of GO:0021700; is a type of synapse organization [GO:0050808]; is part of nervous system development [GO:0007399]